{
  "term_label": "regulation of cell shape",
  "term_id": "GO:0008360",
  "gene_symbol": "FAM171A1",
  "gene_name": "Protein FAM171A1",
  "gene": "UniProtKB:Q5VUB5"
}